{
  "gene": "UniProtKB:Q9UHX1",
  "gene_name": "Poly(U)-binding-splicing factor PUF60",
  "gene_symbol": "PUF60",
  "term_label": "mRNA splice site recognition",
  "term_id": "GO:0006376"
}